{
  "gene_symbol": "CCNA1",
  "gene_name": "Cyclin-A1",
  "gene": "UniProtKB:P78396",
  "term_id": "GO:0005815",
  "term_label": "microtubule organizing center"
}